{
  "gene_name": "Huntingtin-interacting protein 1-related protein",
  "gene": "UniProtKB:O75146",
  "term_id": "GO:0032051",
  "gene_symbol": "HIP1R",
  "term_label": "clathrin light chain binding"
}